{
  "gene": "UniProtKB:Q9HCT0",
  "gene_name": "Fibroblast growth factor 22",
  "term_id": "GO:0005737",
  "gene_symbol": "FGF22",
  "term_label": "cytoplasm"
}